COPII-coated vesicle cargo loading [GO:0090110] (BP) Definition: The formation of a macromolecular complex between the COPII coat proteins and proteins and/or lipoproteins that are going to be transported by the COPII vesicle to the Golgi. Sources: GOC:ascb_2009, GOC:dph, GOC:lb, GOC:tb Also known as: cargo loading into COPII vesicle, cargo loading into COPII-coated vesicle, cargo selection into COPII-coated vesicle, COPII coat-cargo complex assembly Relationships: is a type of vesicle cargo loading [GO:0035459]; is a type of intracellular transport [GO:0046907]; is part of COPII-coated vesicle budding [GO:0090114] Regulation: regulated by regulation of cargo loading into COPII-coated vesicle [GO:1901301]; RO_0002212 by negative regulation of cargo loading into COPII-coated vesicle [GO:1901303]